{
  "gene_symbol": "FDX1",
  "gene_name": "Adrenodoxin, mitochondrial",
  "term_label": "electron transport chain",
  "gene": "UniProtKB:P10109",
  "term_id": "GO:0022900"
}